{
  "gene_symbol": "TXN2",
  "gene": "UniProtKB:Q99757",
  "gene_name": "Thioredoxin, mitochondrial",
  "term_id": "GO:0005739",
  "term_label": "mitochondrion"
}